{
  "gene_symbol": "RELT",
  "term_label": "Unknown molecular function",
  "term_id": "UNKNOWN:0001",
  "gene_name": "Tumor necrosis factor receptor superfamily member 19L",
  "gene": "UniProtKB:Q969Z4"
}